{
  "gene_name": "MAP6 domain-containing protein 1",
  "gene_symbol": "MAP6D1",
  "gene": "UniProtKB:Q9H9H5",
  "term_label": "cis-Golgi network",
  "term_id": "GO:0005801"
}